{
  "term_id": "GO:0005737",
  "gene_symbol": "PSME3",
  "term_label": "cytoplasm",
  "gene": "UniProtKB:P61289",
  "gene_name": "Proteasome activator complex subunit 3"
}